{
  "gene": "UniProtKB:O60907",
  "term_id": "GO:0003714",
  "gene_name": "F-box-like_WD repeat-containing protein TBL1X",
  "term_label": "transcription corepressor activity",
  "gene_symbol": "TBL1X"
}